integrin alpha4-beta7 complex [GO:0034669] (cellular component) References: PMID:12297042 Relationships: is a type of integrin complex [GO:0008305] Definition: An integrin complex that comprises one alpha4 subunit and one beta7 subunit. Also known as: alpha4-beta7 integrin complex, ITGA4-ITGB7 complex